5,6,7,8-tetrahydromethanopterin biosynthetic process [GO:1901285] (biological process) Definition: The chemical reactions and pathways resulting in the formation of 5,6,7,8-tetrahydromethanopterin. Sources: GOC:TermGenie, GOC:yaf, UniPathway:UPA00065 Also known as: 5,6,7,8-tetrahydromethanopterin anabolism, 5,6,7,8-tetrahydromethanopterin biosynthesis, 5,6,7,8-tetrahydromethanopterin formation, 5,6,7,8-tetrahydromethanopterin synthesis Relationships: is_a dicarboxylic acid biosynthetic process [GO:0043650]; is a type of GO:2001118